{
  "term_id": "GO:0001725",
  "gene_name": "LIM domain-binding protein 3",
  "term_label": "stress fiber",
  "gene_symbol": "LDB3",
  "gene": "UniProtKB:O75112"
}